{
  "term_id": "GO:0019957",
  "gene_symbol": "ACKR2",
  "term_label": "C-C chemokine binding",
  "gene_name": "Atypical chemokine receptor 2",
  "gene": "UniProtKB:O00590"
}